{
  "term_label": "DNA-binding transcription factor activity, RNA polymerase II-specific",
  "term_id": "GO:0000981",
  "gene_name": "Transcription factor 23",
  "gene": "UniProtKB:Q7RTU1",
  "gene_symbol": "TCF23"
}